RNA export from nucleus [GO:0006405] (biological process) Relationships: is a type of GO:0050658; is a type of nuclear export [GO:0051168] Also known as: RNA export from cell nucleus, RNA export out of nucleus, RNA transport from nucleus to cytoplasm, RNA-nucleus export Sources: GOC:ma Definition: The directed movement of RNA from the nucleus to the cytoplasm. Subtypes: mRNA export from nucleus [GO:0006406], GO:0006408, tRNA export from nucleus [GO:0006409], GO:0035281, GO:0061716 Regulation: regulated by GO:0046831; negatively regulated by negative regulation of RNA export from nucleus [GO:0046832]; RO_0002213 by positive regulation of RNA export from nucleus [GO:0046833]